sternite morphogenesis [GO:0007491] (biological process) Definition: The process in which the anatomical structures of the sternite are generated and organized. The sternite is the plate or sclerite on the underside of a body segment. References: PMID:16451739 Sources: GOC:jid Relationships: is_a GO:0009886; is part of histoblast morphogenesis [GO:0007488]